activin responsive factor complex [GO:0032444] (cellular component) References: PMID:12374795, PMID:9288972 Also known as: ARF complex Definition: A transcriptionally active complex that binds to an activin response element (ARE) in the promoter of target genes, and is composed of two SMAD2 proteins, one SMAD4 protein and a Forkhead activin signal transducer (FAST) transcription factor. Note: Note that this term should not be confused with any of the molecular function and biological process terms that refer to the small GTPase ARF (ADP-ribosylation factor). Relationships: is a type of RNA polymerase II transcription regulator complex [GO:0090575]